{
  "term_id": "UNKNOWN:0001",
  "term_label": "Unknown molecular function",
  "gene_symbol": "IGKV1-12",
  "gene": "UniProtKB:A0A0C4DH73",
  "gene_name": "Immunoglobulin kappa variable 1-12"
}